{
  "gene_name": "Kinase suppressor of Ras 1",
  "term_id": "GO:0007265",
  "gene_symbol": "KSR1",
  "term_label": "Ras protein signal transduction",
  "gene": "UniProtKB:Q8IVT5"
}